{
  "gene_symbol": "DEPDC5",
  "gene_name": "GATOR complex protein DEPDC5",
  "term_label": "cellular response to amino acid starvation",
  "gene": "UniProtKB:O75140",
  "term_id": "GO:0034198"
}